{
  "gene_symbol": "ZCCHC3",
  "gene": "UniProtKB:Q9NUD5",
  "term_label": "positive regulation of RIG-I signaling pathway",
  "term_id": "GO:1900246",
  "gene_name": "Zinc finger CCHC domain-containing protein 3"
}